{
  "gene": "UniProtKB:Q0IIN9",
  "term_id": "UNKNOWN:0003",
  "term_label": "Unknown cellular component",
  "gene_name": "Putative uncharacterized protein ZNF252P-AS1",
  "gene_symbol": "ZNF252P-AS1"
}